{
  "term_id": "GO:0030154",
  "gene": "UniProtKB:O15105",
  "gene_name": "Mothers against decapentaplegic homolog 7",
  "term_label": "cell differentiation",
  "gene_symbol": "SMAD7"
}